{
  "term_label": "intracellular protein transport",
  "gene": "UniProtKB:P53365",
  "gene_name": "Arfaptin-2",
  "term_id": "GO:0006886",
  "gene_symbol": "ARFIP2"
}